{
  "term_label": "cardiac muscle cell action potential involved in contraction",
  "gene_symbol": "SCN8A",
  "gene": "UniProtKB:Q9UQD0",
  "gene_name": "Sodium channel protein type 8 subunit alpha",
  "term_id": "GO:0086002"
}